{
  "gene_symbol": "IQCF3",
  "term_label": "Unknown cellular component",
  "gene_name": "IQ domain-containing protein F3",
  "term_id": "UNKNOWN:0003",
  "gene": "UniProtKB:P0C7M6"
}